{
  "gene_name": "TELO2-interacting protein 2",
  "gene_symbol": "TTI2",
  "gene": "UniProtKB:Q6NXR4",
  "term_label": "Unknown biological process",
  "term_id": "UNKNOWN:0002"
}